response to risperidone [GO:0097336] (biological process) Sources: GOC:pr Definition: Any process that results in a change in state or activity of a cell or an organism (in terms of movement, secretion, enzyme production, gene expression, etc.) as a result of a risperidone stimulus. Relationships: is a type of GO:1901698; is a type of response to oxygen-containing compound [GO:1901700]